{
  "term_label": "RNA polymerase II cis-regulatory region sequence-specific DNA binding",
  "gene_name": "Transcriptional repressor RHIT",
  "term_id": "GO:0000978",
  "gene": "UniProtKB:O95201",
  "gene_symbol": "ZNF205"
}